{
  "term_id": "GO:0031091",
  "term_label": "platelet alpha granule",
  "gene_symbol": "F5",
  "gene_name": "Coagulation factor V",
  "gene": "UniProtKB:P12259"
}